{
  "term_id": "GO:0016567",
  "term_label": "protein ubiquitination",
  "gene_symbol": "UBD",
  "gene_name": "Ubiquitin D",
  "gene": "UniProtKB:O15205"
}